{
  "gene_name": "Retinal-specific phospholipid-transporting ATPase ABCA4",
  "gene": "UniProtKB:P78363",
  "term_label": "phospholipid transporter activity",
  "term_id": "GO:0005548",
  "gene_symbol": "ABCA4"
}